{
  "term_label": "BMP receptor complex",
  "gene_symbol": "ACVR1",
  "gene_name": "Activin receptor type-1",
  "term_id": "GO:0070724",
  "gene": "UniProtKB:Q04771"
}